{
  "term_id": "UNKNOWN:0001",
  "gene_name": "Vacuolar protein sorting-associated protein 45",
  "term_label": "Unknown molecular function",
  "gene": "UniProtKB:Q9NRW7",
  "gene_symbol": "VPS45"
}